regulation of flocculation [GO:0060256] (biological process) Also known as: regulation of flocculation via cell wall protein-carbohydrate interaction References: PMID:10591965, PMID:15466424, PMID:16568252 Relationships: is a type of regulation of cell-cell adhesion [GO:0022407]; regulates flocculation [GO:0000128] Definition: Any process that modulates the rate, frequency or extent of the non-sexual aggregation of single-celled organisms. Subtypes: negative regulation of flocculation [GO:0060257], positive regulation of flocculation [GO:1900735]